positive regulation of macromolecule metabolic process [GO:0010604] (biological process) Sources: GOC:dph, GOC:tb Subtypes: positive regulation of receptor recycling [GO:0001921], positive regulation of macromolecule biosynthetic process [GO:0010557], positive regulation of DNA metabolic process [GO:0051054], GO:0051247, positive regulation of RNA metabolic process [GO:0051254], positive regulation of glycogen metabolic process [GO:0070875], GO:2000646, positive regulation of starch catabolic process [GO:2000883], positive regulation of galactoglucomannan catabolic process [GO:2000914], positive regulation of cellodextrin catabolic process [GO:2000929], positive regulation of cyclodextrin catabolic process [GO:2000959], GO:2000968, positive regulation of hemicellulose catabolic process [GO:2000990], positive regulation of galactomannan catabolic process [GO:2000993], positive regulation of cellulose catabolic process [GO:2000999], positive regulation of pectin catabolic process [GO:2001005] Definition: Any process that increases the frequency, rate or extent of the chemical reactions and pathways involving macromolecules, any molecule of high relative molecular mass, the structure of which essentially comprises the multiple repetition of units derived, actually or conceptually, from molecules of low relative molecular mass. Relationships: is a type of positive regulation of metabolic process [GO:0009893]; is a type of GO:0060255; positively regulates GO:0043170